{
  "term_label": "mRNA binding",
  "term_id": "GO:0003729",
  "gene_symbol": "SRSF3",
  "gene": "UniProtKB:P84103",
  "gene_name": "Serine_arginine-rich splicing factor 3"
}